{
  "gene": "UniProtKB:P05112",
  "gene_name": "Interleukin-4",
  "term_label": "Unknown cellular component",
  "gene_symbol": "IL4",
  "term_id": "UNKNOWN:0003"
}